endothelial differentiation G protein-coupled receptor binding [GO:0031753] (molecular function) Definition: Binding to an endothelial differentiation G protein-coupled receptor. Sources: GOC:mah, GOC:nln Also known as: endothelial differentiation G-protein coupled receptor binding, endothelial differentiation G-protein coupled receptor ligand Relationships: is a type of G protein-coupled receptor binding [GO:0001664] Subtypes: Edg-1 sphingosine 1-phosphate receptor binding [GO:0031754], GO:0031755, Edg-3 sphingosine 1-phosphate receptor binding [GO:0031756], Edg-4 lysophosphatidic acid receptor binding [GO:0031757], Edg-5 sphingosine 1-phosphate receptor binding [GO:0031758], Edg-6 sphingosine 1-phosphate receptor binding [GO:0031759], GO:0031760